negative regulation of substance P secretion [GO:1904459] (biological process) Subtypes: GO:1904495 Also known as: down regulation of substance P secretion, down-regulation of substance P secretion, downregulation of substance P secretion, inhibition of substance P secretion References: PMID:11278900 Sources: GOC:TermGenie, GO_REF:0000058 Relationships: is a type of negative regulation of peptide hormone secretion [GO:0090278]; is a type of regulation of substance P secretion [GO:1904458]; negatively regulates GO:1990772 Definition: Any process that stops, prevents or reduces the frequency, rate or extent of substance P secretion.